{
  "term_label": "vacuolar membrane",
  "gene_symbol": "NPRL2",
  "gene": "UniProtKB:Q8WTW4",
  "term_id": "GO:0005774",
  "gene_name": "GATOR complex protein NPRL2"
}